diet induced thermogenesis [GO:0002024] (biological process) Definition: The process that results in increased metabolic rate in tissues of an organism. It is triggered by the detection of dietary excess. This process is achieved via signaling in the sympathetic nervous system. References: PMID:12161655 Relationships: is a type of adaptive thermogenesis [GO:1990845]; is part of response to dietary excess [GO:0002021]